{
  "term_label": "Unknown biological process",
  "term_id": "UNKNOWN:0002",
  "gene_name": "Putative uncharacterized protein encoded by LINC00322",
  "gene": "UniProtKB:Q6ZN03",
  "gene_symbol": "LINC00322"
}